{
  "term_id": "GO:0006888",
  "term_label": "endoplasmic reticulum to Golgi vesicle-mediated transport",
  "gene": "UniProtKB:O43264",
  "gene_name": "Centromere_kinetochore protein zw10 homolog",
  "gene_symbol": "ZW10"
}